CD8-positive, alpha-beta T cell differentiation involved in immune response [GO:0002302] (biological process) Definition: The process in which an antigenically naive CD8-positive, alpha-beta T cell acquires the specialized features of an effector, regulatory, or memory T cell as part of an immune response. Effector T cells include cells which provide T cell help or exhibit cytotoxicity towards other cells. Note: Note that immunologists typically use the word 'development' to refer to cells of B or T cell lineages undergoing the process that GO describes as 'cell differentiation'. Also known as: CD8-positive, alpha-beta T cell differentiation during immune response, CD8-positive, alpha-beta T lymphocyte differentiation during immune response, CD8-positive, alpha-beta T-cell differentiation during immune response, CD8-positive, alpha-beta T-lymphocyte differentiation during immune response, CD8-positive, alpha-beta intraepithelial T cell development Sources: GOC:add, ISBN:0781735149 Relationships: is a type of alpha-beta T cell differentiation involved in immune response [GO:0002293]; is a type of CD8-positive, alpha-beta T cell differentiation [GO:0043374]